{
  "gene_symbol": "ZNF445",
  "gene_name": "Zinc finger protein 445",
  "term_label": "regulation of transcription by RNA polymerase II",
  "term_id": "GO:0006357",
  "gene": "UniProtKB:P59923"
}